{
  "term_label": "Unknown molecular function",
  "gene_name": "Coiled-coil domain-containing protein R3HCC1L",
  "term_id": "UNKNOWN:0001",
  "gene_symbol": "R3HCC1L",
  "gene": "UniProtKB:Q7Z5L2"
}